{
  "gene": "UniProtKB:A0A0C4DH33",
  "gene_symbol": "IGHV1-24",
  "term_label": "immunoglobulin mediated immune response",
  "term_id": "GO:0016064",
  "gene_name": "Immunoglobulin heavy variable 1-24"
}